{
  "gene": "UniProtKB:Q969N2",
  "term_id": "UNKNOWN:0001",
  "gene_name": "GPI transamidase component PIG-T",
  "gene_symbol": "PIGT",
  "term_label": "Unknown molecular function"
}